venom-mediated vasodilation by activation of nitric oxide-cGMP-mediated signaling [GO:0140165] (biological process) Also known as: venom-mediated vasodilation induced by nitric oxide activity References: PMID:10512636 Relationships: is a type of venom-mediated perturbation of signal transduction [GO:0044509]; is a type of venom-mediated vasodilation [GO:0044551] Definition: A process in which an organism initiates, promotes, or enhances vasodilation via the action of a venom that activates nitric oxide-cGMP-mediated signaling, concomittantly reducing blood pressure in the bitten/stung organism.